{
  "term_id": "GO:0007186",
  "gene": "UniProtKB:Q8NGE9",
  "term_label": "G protein-coupled receptor signaling pathway",
  "gene_symbol": "OR9Q2",
  "gene_name": "Olfactory receptor 9Q2"
}